{
  "term_label": "cell morphogenesis involved in neuron differentiation",
  "gene": "UniProtKB:P06400",
  "gene_name": "Retinoblastoma-associated protein",
  "term_id": "GO:0048667",
  "gene_symbol": "RB1"
}